{
  "term_id": "GO:0051787",
  "gene_symbol": "DNAJC10",
  "term_label": "misfolded protein binding",
  "gene": "UniProtKB:Q8IXB1",
  "gene_name": "DnaJ homolog subfamily C member 10"
}